{
  "term_id": "GO:0003844",
  "gene_symbol": "GBE1",
  "gene_name": "1,4-alpha-glucan-branching enzyme",
  "gene": "UniProtKB:Q04446",
  "term_label": "1,4-alpha-glucan branching enzyme activity"
}